{
  "gene_name": "Alpha-mannosidase 2x",
  "gene": "UniProtKB:P49641",
  "term_id": "GO:0006491",
  "gene_symbol": "MAN2A2",
  "term_label": "N-glycan processing"
}